{
  "gene_name": "Rabphilin-3A",
  "gene": "UniProtKB:Q9Y2J0",
  "term_id": "GO:0045956",
  "gene_symbol": "RPH3A",
  "term_label": "positive regulation of calcium ion-dependent exocytosis"
}